{
  "gene_name": "RNA-binding E3 ubiquitin-protein ligase MEX3C",
  "term_label": "Unknown biological process",
  "gene": "UniProtKB:Q5U5Q3",
  "term_id": "UNKNOWN:0002",
  "gene_symbol": "MEX3C"
}